{
  "gene": "UniProtKB:O60479",
  "gene_name": "Homeobox protein DLX-3",
  "term_label": "embryonic skeletal system development",
  "term_id": "GO:0048706",
  "gene_symbol": "DLX3"
}